{
  "gene_symbol": "CDX2",
  "gene_name": "Homeobox protein CDX-2",
  "term_label": "digestive tract development",
  "gene": "UniProtKB:Q99626",
  "term_id": "GO:0048565"
}